{
  "term_label": "neurogenesis",
  "gene_symbol": "FGF19",
  "gene_name": "Fibroblast growth factor 19",
  "gene": "UniProtKB:O95750",
  "term_id": "GO:0022008"
}